{
  "gene_symbol": "MTR",
  "term_id": "GO:0009086",
  "gene_name": "Methionine synthase",
  "term_label": "methionine biosynthetic process",
  "gene": "UniProtKB:Q99707"
}